regulation of ferricrocin biosynthetic process [GO:1900678] (biological process) Definition: Any process that modulates the frequency, rate or extent of ferricrocin biosynthetic process. Sources: GOC:TermGenie, GOC:di Also known as: regulation of ferricrocin anabolism, regulation of ferricrocin biosynthesis, regulation of ferricrocin formation, regulation of ferricrocin synthesis, regulation of ferricrocin biosynthetic process, peptide formation, regulation of ferricrocin biosynthetic process, peptide modification Relationships: is a type of regulation of ferrichrome biosynthetic process [GO:1905568]; regulates GO:0031171 Subtypes: negative regulation of ferricrocin biosynthetic process [GO:1900679], positive regulation of ferricrocin biosynthetic process [GO:1900680]